{
  "gene_name": "F-box only protein 11",
  "gene": "UniProtKB:Q86XK2",
  "term_id": "GO:0006511",
  "gene_symbol": "FBXO11",
  "term_label": "ubiquitin-dependent protein catabolic process"
}